{
  "term_id": "GO:0000981",
  "gene": "UniProtKB:Q9UL36",
  "gene_symbol": "ZNF236",
  "gene_name": "Zinc finger protein 236",
  "term_label": "DNA-binding transcription factor activity, RNA polymerase II-specific"
}